{
  "gene_name": "Diacylglycerol lipase-alpha",
  "term_label": "postsynaptic membrane",
  "gene_symbol": "DAGLA",
  "term_id": "GO:0045211",
  "gene": "UniProtKB:Q9Y4D2"
}